{
  "term_id": "GO:0030334",
  "gene_name": "Fibroblast growth factor 1",
  "term_label": "regulation of cell migration",
  "gene": "UniProtKB:P05230",
  "gene_symbol": "FGF1"
}